{
  "term_id": "GO:0060828",
  "gene_symbol": "PTK7",
  "term_label": "regulation of canonical Wnt signaling pathway",
  "gene_name": "Inactive tyrosine-protein kinase 7",
  "gene": "UniProtKB:Q13308"
}